{
  "gene_name": "Mitotic-spindle organizing protein 1",
  "gene_symbol": "MZT1",
  "term_label": "interphase microtubule organizing center",
  "gene": "UniProtKB:Q08AG7",
  "term_id": "GO:0031021"
}